{
  "gene_symbol": "FLT4",
  "term_label": "positive regulation of cell migration",
  "gene_name": "Vascular endothelial growth factor receptor 3",
  "gene": "UniProtKB:P35916",
  "term_id": "GO:0030335"
}